{
  "term_label": "Unknown cellular component",
  "gene": "UniProtKB:Q3SY05",
  "term_id": "UNKNOWN:0003",
  "gene_symbol": "LINC00303",
  "gene_name": "Putative uncharacterized protein encoded by LINC00303"
}